{
  "gene_symbol": "SHISA9",
  "term_id": "GO:0048172",
  "gene": "UniProtKB:B4DS77",
  "term_label": "regulation of short-term neuronal synaptic plasticity",
  "gene_name": "Protein shisa-9"
}